{
  "gene_name": "Bardet-Biedl syndrome 4 protein",
  "term_id": "GO:0061512",
  "gene": "UniProtKB:Q96RK4",
  "gene_symbol": "BBS4",
  "term_label": "protein localization to cilium"
}